{
  "gene": "UniProtKB:O00141",
  "gene_symbol": "SGK1",
  "gene_name": "Serine_threonine-protein kinase Sgk1",
  "term_id": "GO:0004674",
  "term_label": "protein serine/threonine kinase activity"
}